negative regulation of glial cell migration [GO:1903976] (biological process) Definition: Any process that stops, prevents or reduces the frequency, rate or extent of glial cell migration. References: PMID:19100238 Sources: GOC:BHF, GOC:TermGenie, GOC:nc, GO_REF:0000058 Also known as: down regulation of glia cell migration, down regulation of glial cell migration, down-regulation of glia cell migration, down-regulation of glial cell migration, downregulation of glia cell migration, downregulation of glial cell migration, negative regulation of glia cell migration, inhibition of glia cell migration, inhibition of glial cell migration Relationships: is a type of negative regulation of cell migration [GO:0030336]; is a type of GO:1903975; negatively regulates GO:0008347 Subtypes: negative regulation of cell motility involved in cerebral cortex radial glia guided migration [GO:0021822], negative regulation of Schwann cell migration [GO:1900148], GO:1904140, negative regulation of astrocyte chemotaxis [GO:2000459]